{
  "term_id": "GO:0006357",
  "gene_symbol": "ZSCAN23",
  "gene_name": "Zinc finger and SCAN domain-containing protein 23",
  "term_label": "regulation of transcription by RNA polymerase II",
  "gene": "UniProtKB:Q3MJ62"
}